eosinophil migration [GO:0072677] (biological process) Definition: The movement of an eosinophil within or between different tissues and organs of the body. Sources: CL:0000771, GOC:BHF, GOC:mah Relationships: is a type of granulocyte migration [GO:0097530] Subtypes: eosinophil chemotaxis [GO:0048245], eosinophil extravasation [GO:0072682] Regulation: RO_0002211 by regulation of eosinophil migration [GO:2000416]; negatively regulated by negative regulation of eosinophil migration [GO:2000417]; positively regulated by positive regulation of eosinophil migration [GO:2000418]